{
  "gene_symbol": "APRG1",
  "gene_name": "APRG1 tumor suppressor candidate",
  "term_label": "Unknown biological process",
  "gene": "UniProtKB:Q8IVJ8",
  "term_id": "UNKNOWN:0002"
}